{
  "gene": "UniProtKB:O75817",
  "gene_symbol": "POP7",
  "term_id": "UNKNOWN:0001",
  "gene_name": "Ribonuclease P protein subunit p20",
  "term_label": "Unknown molecular function"
}